{
  "gene_name": "Bifunctional purine biosynthesis protein ATIC",
  "gene_symbol": "ATIC",
  "term_label": "'de novo' IMP biosynthetic process",
  "gene": "UniProtKB:P31939",
  "term_id": "GO:0006189"
}